ethanolamine ammonia-lyase activity [GO:0008851] (molecular function) Also known as: ethanolamine ammonia-lyase (acetaldehyde-forming) activity, ethanolamine deaminase activity Relationships: is a type of ammonia-lyase activity [GO:0016841] Sources: EC:4.3.1.7 Definition: Catalysis of the reaction: ethanolamine = acetaldehyde + NH3.